{
  "gene_symbol": "PM20D2",
  "term_label": "dipeptidase activity",
  "gene_name": "Xaa-Arg dipeptidase",
  "gene": "UniProtKB:Q8IYS1",
  "term_id": "GO:0016805"
}